{
  "gene": "UniProtKB:Q9UHW9",
  "term_label": "plasma membrane",
  "term_id": "GO:0005886",
  "gene_symbol": "SLC12A6",
  "gene_name": "Solute carrier family 12 member 6"
}